negative regulation of phosphorylation [GO:0042326] (biological process) Relationships: is a type of regulation of phosphorylation [GO:0042325]; is a type of negative regulation of phosphate metabolic process [GO:0045936]; negatively regulates GO:0016310 Sources: GOC:jl Also known as: down regulation of phosphorylation, down-regulation of phosphorylation, downregulation of phosphorylation, inhibition of phosphorylation Subtypes: negative regulation of protein phosphorylation [GO:0001933], GO:0033673 Note: Note that this term is in the subset of terms that should not be used for direct gene product annotation. Instead, select a child term or, if no appropriate child term exists, please request a new term. Direct annotations to this term may be amended during annotation QC. Definition: Any process that stops, prevents or decreases the rate of addition of phosphate groups to a molecule.